{
  "gene": "UniProtKB:Q9UBN4",
  "term_id": "GO:0015279",
  "gene_symbol": "TRPC4",
  "term_label": "store-operated calcium channel activity",
  "gene_name": "Short transient receptor potential channel 4"
}